{
  "term_id": "GO:0006357",
  "term_label": "regulation of transcription by RNA polymerase II",
  "gene": "UniProtKB:Q5VV52",
  "gene_name": "Zinc finger protein 691",
  "gene_symbol": "ZNF691"
}